positive regulation of T cell activation via T cell receptor contact with antigen bound to MHC molecule on antigen presenting cell [GO:2001190] (BP) Sources: GOC:obol Also known as: positive regulation of T lymphocyte activation via T cell receptor contact with antigen bound to MHC molecule on antigen presenting cell, positive regulation of T-cell activation via T cell receptor contact with antigen bound to MHC molecule on antigen presenting cell, positive regulation of T-lymphocyte activation via T cell receptor contact with antigen bound to MHC molecule on antigen presenting cell Relationships: is a type of GO:0002699; is a type of positive regulation of immune response [GO:0050778]; is a type of positive regulation of T cell activation [GO:0050870]; is a type of regulation of T cell activation via T cell receptor contact with antigen bound to MHC molecule on antigen presenting cell [GO:2001188]; positively regulates T cell activation via T cell receptor contact with antigen bound to MHC molecule on antigen presenting cell [GO:0002291] Definition: Any process that activates or increases the frequency, rate or extent of T cell activation via T cell receptor contact with antigen bound to MHC molecule on antigen presenting cell.